{
  "term_label": "postsynaptic density",
  "gene": "UniProtKB:Q9UEY8",
  "gene_name": "Gamma-adducin",
  "term_id": "GO:0014069",
  "gene_symbol": "ADD3"
}